{
  "term_label": "mitotic DNA replication checkpoint signaling",
  "term_id": "GO:0033314",
  "gene": "UniProtKB:Q8NHY5",
  "gene_name": "Checkpoint protein HUS1B",
  "gene_symbol": "HUS1B"
}